{
  "term_label": "glycogenin glucosyltransferase activity",
  "gene_name": "Glycogenin-2",
  "gene_symbol": "GYG2",
  "gene": "UniProtKB:O15488",
  "term_id": "GO:0008466"
}